regulation of dCDP biosynthetic process [GO:1903528] (biological process) Subtypes: negative regulation of dCDP biosynthetic process [GO:1903529] Definition: Any process that modulates the frequency, rate or extent of dCDP biosynthetic process. References: PMID:16317005 Sources: GOC:TermGenie, GO_REF:0000058 Relationships: is a type of regulation of pyrimidine nucleotide biosynthetic process [GO:1900397]; regulates dCDP biosynthetic process [GO:0006240] Also known as: regulation of dCDP anabolism, regulation of dCDP biosynthesis, regulation of dCDP formation, regulation of dCDP synthesis